{
  "gene": "UniProtKB:O95976",
  "term_id": "UNKNOWN:0002",
  "gene_name": "Immunoglobulin superfamily member 6",
  "term_label": "Unknown biological process",
  "gene_symbol": "IGSF6"
}